{
  "term_label": "extracellular matrix structural constituent conferring tensile strength",
  "gene": "UniProtKB:Q02388",
  "gene_symbol": "COL7A1",
  "gene_name": "Collagen alpha-1(VII) chain",
  "term_id": "GO:0030020"
}